{
  "gene_symbol": "ZNF3",
  "gene_name": "Zinc finger protein 3",
  "gene": "UniProtKB:P17036",
  "term_id": "GO:0000977",
  "term_label": "RNA polymerase II transcription regulatory region sequence-specific DNA binding"
}